{
  "gene_symbol": "PRR7",
  "term_id": "GO:0005634",
  "term_label": "nucleus",
  "gene_name": "Proline-rich protein 7",
  "gene": "UniProtKB:Q8TB68"
}